intra-Golgi vesicle-mediated transport [GO:0006891] (biological process) Also known as: intra-Golgi transport Sources: ISBN:0716731363 Definition: The directed movement of substances within the Golgi, mediated by small transport vesicles. These either fuse with the cis-Golgi or with each other to form the membrane stacks known as the cis-Golgi reticulum (network). Subtypes: retrograde transport, vesicle recycling within Golgi [GO:0000301], GO:0045057, inter-Golgi cisterna vesicle-mediated transport [GO:0048219] Relationships: is a type of Golgi vesicle transport [GO:0048193]